{
  "gene": "UniProtKB:Q14119",
  "term_id": "GO:0000977",
  "gene_symbol": "VEZF1",
  "term_label": "RNA polymerase II transcription regulatory region sequence-specific DNA binding",
  "gene_name": "Vascular endothelial zinc finger 1"
}